{
  "gene_name": "Keratin-associated protein 16-1",
  "gene": "UniProtKB:A8MUX0",
  "term_id": "UNKNOWN:0001",
  "term_label": "Unknown molecular function",
  "gene_symbol": "KRTAP16-1"
}